determinate inflorescence morphogenesis [GO:0048282] (biological process) Definition: The process in which the anatomical structures of determinate inflorescences are generated and organized. A determinate inflorescence is one that can only produce a predetermined number of floral meristems. References: PMID:9553044 Sources: GOC:jid Relationships: is a type of inflorescence morphogenesis [GO:0048281]